{
  "term_label": "positive regulation of transcription by RNA polymerase II",
  "term_id": "GO:0045944",
  "gene_symbol": "CASZ1",
  "gene": "UniProtKB:Q86V15",
  "gene_name": "Zinc finger protein castor homolog 1"
}